{
  "term_label": "intracellular signal transduction",
  "term_id": "GO:0035556",
  "gene": "UniProtKB:P49137",
  "gene_symbol": "MAPKAPK2",
  "gene_name": "MAP kinase-activated protein kinase 2"
}